{
  "term_id": "GO:0008284",
  "gene": "UniProtKB:A6NDR6",
  "gene_name": "Putative homeobox protein Meis3-like 1",
  "gene_symbol": "MEIS3P1",
  "term_label": "positive regulation of cell population proliferation"
}